{
  "gene_name": "DNA repair protein RAD51 homolog 2",
  "gene_symbol": "RAD51B",
  "term_label": "double-stranded DNA binding",
  "term_id": "GO:0003690",
  "gene": "UniProtKB:O15315"
}